glucuronan lyase activity [GO:0033994] (molecular function) Definition: Catalysis of the reaction: (1->4)-beta-D-glucuronan = an oligosaccharide with 4-deoxy-beta-D-gluc-4-enuronosyl end + (1->4)-beta-D-glucuronan. This reaction is the eliminative cleavage of (1->4)-beta-D-glucuronans to give oligosaccharides with 4-deoxy-beta-D-gluc-4-enuronosyl groups at their non-reducing ends. Complete degradation of glucuronans results in the formation of tetrasaccharides. Sources: EC:4.2.2.14 Also known as: (1,4)-beta-D-glucuronan lyase activity Relationships: is a type of carbon-oxygen lyase activity, acting on polysaccharides [GO:0016837]